{
  "gene_name": "Voltage-dependent T-type calcium channel subunit alpha-1I",
  "gene_symbol": "CACNA1I",
  "gene": "UniProtKB:Q9P0X4",
  "term_id": "GO:0098703",
  "term_label": "calcium ion import across plasma membrane"
}